{
  "gene_symbol": "OR52E5",
  "gene_name": "Olfactory receptor 52E5",
  "gene": "UniProtKB:Q8NH55",
  "term_id": "GO:0004984",
  "term_label": "olfactory receptor activity"
}